{
  "gene_symbol": "CSF3",
  "gene": "UniProtKB:P09919",
  "gene_name": "Granulocyte colony-stimulating factor",
  "term_label": "extracellular space",
  "term_id": "GO:0005615"
}